{
  "term_label": "Unknown molecular function",
  "gene_name": "Tastin",
  "gene": "UniProtKB:Q12815",
  "term_id": "UNKNOWN:0001",
  "gene_symbol": "TROAP"
}